chromaffin granule membrane [GO:0042584] (cellular component) Sources: GOC:jl Definition: The lipid bilayer surrounding a chromaffin granule, a specialized secretory vesicle found in the cells of adrenal glands and various other organs, which is concerned with the synthesis, storage, metabolism, and secretion of epinephrine and norepinephrine. Relationships: is a type of secretory granule membrane [GO:0030667]; is part of GO:0042583